{
  "term_label": "monoatomic cation transport",
  "gene_symbol": "PANX1",
  "term_id": "GO:0006812",
  "gene_name": "Pannexin-1",
  "gene": "UniProtKB:Q96RD7"
}